{
  "term_id": "GO:0106435",
  "gene_name": "Carboxylesterase 3",
  "term_label": "carboxylesterase activity",
  "gene_symbol": "CES3",
  "gene": "UniProtKB:Q6UWW8"
}